double fertilization forming a zygote and endosperm [GO:0009567] (biological process) Also known as: double fertilization Sources: GOC:mtg_sensu, GOC:tb Definition: Fertilization where one of the two sperm nuclei from the pollen tube fuses with the egg nucleus to form a 2n zygote, and the other fuses with the two polar nuclei to form the 3n primary endosperm nucleus and then develops into the endosperm. The ploidy level of the 2n zygote and 3n primary endosperm nucleus is determined by the ploidy level of the parents involved. An example of this component is found in Arabidopsis thaliana. Regulation: regulated by regulation of double fertilization forming a zygote and endosperm [GO:0080155] Relationships: is_a GO:0009566